{
  "gene_symbol": "HAPLN3",
  "gene_name": "Hyaluronan and proteoglycan link protein 3",
  "term_id": "GO:0005615",
  "gene": "UniProtKB:Q96S86",
  "term_label": "extracellular space"
}